{
  "term_label": "RNA polymerase II cis-regulatory region sequence-specific DNA binding",
  "term_id": "GO:0000978",
  "gene_symbol": "STAT6",
  "gene_name": "Signal transducer and activator of transcription 6",
  "gene": "UniProtKB:P42226"
}